{
  "term_id": "GO:0047496",
  "term_label": "vesicle transport along microtubule",
  "gene_symbol": "CDR2L",
  "gene_name": "Cerebellar degeneration-related protein 2-like",
  "gene": "UniProtKB:Q86X02"
}